{
  "term_id": "UNKNOWN:0001",
  "gene": "UniProtKB:Q9UHR5",
  "term_label": "Unknown molecular function",
  "gene_symbol": "SAP30BP",
  "gene_name": "SAP30-binding protein"
}